{
  "gene": "UniProtKB:O00635",
  "term_id": "GO:0061630",
  "gene_symbol": "TRIM38",
  "term_label": "ubiquitin protein ligase activity",
  "gene_name": "E3 ubiquitin-protein ligase TRIM38"
}